{
  "term_label": "cytoplasm",
  "gene": "UniProtKB:Q13402",
  "term_id": "GO:0005737",
  "gene_symbol": "MYO7A",
  "gene_name": "Unconventional myosin-VIIa"
}